{
  "term_id": "GO:0007186",
  "gene": "UniProtKB:P49019",
  "term_label": "G protein-coupled receptor signaling pathway",
  "gene_symbol": "HCAR3",
  "gene_name": "Hydroxycarboxylic acid receptor 3"
}